{
  "term_label": "metallocarboxypeptidase activity",
  "gene": "UniProtKB:P15086",
  "gene_name": "Carboxypeptidase B",
  "term_id": "GO:0004181",
  "gene_symbol": "CPB1"
}